{
  "gene_symbol": "OR5H6",
  "gene_name": "Olfactory receptor 5H6",
  "gene": "UniProtKB:Q8NGV6",
  "term_id": "UNKNOWN:0002",
  "term_label": "Unknown biological process"
}